{
  "term_label": "synaptic transmission, GABAergic",
  "gene_name": "Gamma-aminobutyric acid receptor subunit rho-1",
  "term_id": "GO:0051932",
  "gene": "UniProtKB:P24046",
  "gene_symbol": "GABRR1"
}